{
  "gene": "UniProtKB:Q8TE68",
  "gene_symbol": "EPS8L1",
  "term_label": "ruffle membrane",
  "gene_name": "Epidermal growth factor receptor kinase substrate 8-like protein 1",
  "term_id": "GO:0032587"
}